{
  "term_id": "UNKNOWN:0003",
  "gene_symbol": "LRRC71",
  "gene_name": "Leucine-rich repeat-containing protein 71",
  "term_label": "Unknown cellular component",
  "gene": "UniProtKB:Q8N4P6"
}